cysteine-type endopeptidase inhibitor activity [GO:0004869] (molecular function) Definition: Binds to and stops, prevents or reduces the activity of a cysteine-type endopeptidase. Sources: GOC:dph, GOC:tb Also known as: cystatin, cysteine protease inhibitor activity, thiol protease inhibitor Relationships: is a type of endopeptidase inhibitor activity [GO:0004866]; negatively regulates GO:0004197 Subtypes: calcium-dependent cysteine-type endopeptidase inhibitor activity [GO:0010859]